{
  "gene": "UniProtKB:Q96AY2",
  "term_id": "GO:0000712",
  "gene_name": "Crossover junction endonuclease EME1",
  "term_label": "resolution of meiotic recombination intermediates",
  "gene_symbol": "EME1"
}